{
  "gene_name": "DNA replication complex GINS protein PSF3",
  "gene": "UniProtKB:Q9BRX5",
  "term_label": "DNA replication initiation",
  "term_id": "GO:0006270",
  "gene_symbol": "GINS3"
}